{
  "term_label": "single-stranded DNA binding",
  "gene_name": "Aprataxin",
  "term_id": "GO:0003697",
  "gene_symbol": "APTX",
  "gene": "UniProtKB:Q7Z2E3"
}